regulation of microglial cell migration [GO:1904139] (biological process) Definition: Any process that modulates the frequency, rate or extent of microglial cell migration. Relationships: is a type of regulation of glial cell migration [GO:1903975]; is a type of regulation of macrophage migration [GO:1905521]; regulates microglial cell migration [GO:1904124] Subtypes: negative regulation of microglial cell migration [GO:1904140], positive regulation of microglial cell migration [GO:1904141] References: PMID:19100238 Sources: GOC:BHF, GOC:TermGenie, GOC:nc, GO_REF:0000058